{
  "gene_name": "Capping protein, Arp2_3 and myosin-I linker protein 3",
  "term_id": "GO:0030027",
  "gene_symbol": "CARMIL3",
  "term_label": "lamellipodium",
  "gene": "UniProtKB:Q8ND23"
}